anterograde axonal protein transport [GO:0099641] (biological process) Definition: The directed movement of proteins along microtubules from the cell body toward the cell periphery in nerve cell axons. Relationships: is a type of GO:0008089; is a type of GO:0099640; is a type of protein localization to presynapse [GO:1905383] Also known as: anterograde axon cargo transport Sources: GOC:dos Subtypes: GO:0140231